G1 to G0 transition involved in cell differentiation [GO:0070315] (BP) Definition: A cell cycle arrest process that results in arrest during G1 phase, whereupon the cell enters G0 phase, in the context of cell differentiation. Sources: GOC:mah, ISBN:0815316194 Relationships: is a type of G1 to G0 transition [GO:0070314]; is part of cell differentiation [GO:0030154] Also known as: G1/G0 transition involved in cell differentiation